{
  "gene_symbol": "CCL3",
  "term_label": "positive regulation of cell migration",
  "term_id": "GO:0030335",
  "gene_name": "C-C motif chemokine 3",
  "gene": "UniProtKB:P10147"
}